aspyridone A catabolic process [GO:1901517] (biological process) Sources: GOC:TermGenie, GOC:di Also known as: aspyridone A breakdown, aspyridone A catabolism, aspyridone A degradation Relationships: is a type of polyketide catabolic process [GO:0030640]; is a type of pyridine-containing compound catabolic process [GO:0072526] Definition: The chemical reactions and pathways resulting in the breakdown of aspyridone A.